3-hydroxyphenyl propionate:proton symporter activity [GO:0015540] (molecular function) Sources: TC:2.A.1.15.2 Definition: Enables the transfer of a solute or solutes from one side of a membrane to the other according to the reaction: 3-hydroxyphenyl propionate(out) + H+(out) = 3-hydroxyphenyl propionate(in) + H+(in). Relationships: is_a GO:0015295; is_a 3-hydroxyphenyl propanoate transmembrane transporter activity [GO:0015551] Also known as: 3-hydroxyphenyl propionate:hydrogen ion symporter activity, 3-hydroxyphenyl propionate porter activity